{
  "gene_name": "Protein odd-skipped-related 2",
  "gene": "UniProtKB:Q8N2R0",
  "gene_symbol": "OSR2",
  "term_label": "urogenital system development",
  "term_id": "GO:0001655"
}